{
  "term_id": "GO:0005789",
  "gene_name": "Acyl-coenzyme A diphosphatase FITM2",
  "gene": "UniProtKB:Q8N6M3",
  "gene_symbol": "FITM2",
  "term_label": "endoplasmic reticulum membrane"
}